{
  "gene": "UniProtKB:Q96Q45",
  "gene_symbol": "TMEM237",
  "term_id": "GO:0035869",
  "gene_name": "Transmembrane protein 237",
  "term_label": "ciliary transition zone"
}